{
  "term_label": "GTPase activity",
  "gene": "UniProtKB:Q92730",
  "gene_symbol": "RND1",
  "term_id": "GO:0003924",
  "gene_name": "Rho-related GTP-binding protein Rho6"
}